{
  "term_label": "large ribosomal subunit rRNA binding",
  "gene": "UniProtKB:P30050",
  "gene_symbol": "RPL12",
  "term_id": "GO:0070180",
  "gene_name": "Large ribosomal subunit protein uL11"
}